{
  "gene": "UniProtKB:Q2M3G4",
  "gene_symbol": "SHROOM1",
  "gene_name": "Protein Shroom1",
  "term_id": "GO:0051015",
  "term_label": "actin filament binding"
}